{
  "term_id": "GO:0005516",
  "gene_symbol": "RIT2",
  "term_label": "calmodulin binding",
  "gene_name": "GTP-binding protein Rit2",
  "gene": "UniProtKB:Q99578"
}